{
  "gene_symbol": "HSD3B2",
  "term_id": "GO:0008207",
  "gene": "UniProtKB:P26439",
  "term_label": "C21-steroid hormone metabolic process",
  "gene_name": "3 beta-hydroxysteroid dehydrogenase_Delta 5--4-isomerase type 2"
}